spinal cord radial glial cell differentiation [GO:0021531] (biological process) Definition: The process in which neuroepithelial cells in the ventral neural tube acquire specialized structural and/or functional features of radial glial cells. Radial cell precursors differentiate into both neuronal cell types and mature radial glial cells. Mature radial glial cells regulate the axon growth and pathfinding processes that occur during white matter patterning of the developing spinal cord. Differentiation includes the processes involved in commitment of a cell to a specific fate. Relationships: is a type of cell differentiation in spinal cord [GO:0021515]; is a type of radial glial cell differentiation [GO:0060019] Also known as: radial glial cell differentiation in spinal cord References: PMID:16185248 Sources: GOC:cls, GOC:dgh, GOC:dph, GOC:jid, GO_REF:0000021